DNA recombinase disassembly [GO:1990986] (biological process) Relationships: is a type of protein-DNA complex disassembly [GO:0032986] Also known as: Rad51 nucleoprotein filament disassembly Regulation: regulated by regulation of DNA recombinase disassembly [GO:0062109]; negatively regulated by negative regulation of DNA recombinase disassembly [GO:0062110] Definition: The disaggregation of a DNA recombinase complex into its constituent strand exchange proteins (recombinases). References: PMID:19540122 Sources: GOC:pg